detection of biotic stimulus [GO:0009595] (biological process) Definition: The series of events in which a biotic stimulus, one caused or produced by a living organism, is received and converted into a molecular signal. Relationships: is a type of response to biotic stimulus [GO:0009607]; is a type of detection of stimulus [GO:0051606] Subtypes: detection of endoplasmic reticulum overloading [GO:0002234], GO:0002355, GO:0060245, GO:0098581 Sources: GOC:hb Also known as: perception of biotic stimulus